basement membrane [GO:0005604] (cellular component) Also known as: basal lamina, basement lamina, lamina densa Note: Note that this term has no relationship to 'membrane ; GO:0016020' because the basement membrane is not a lipid bilayer. Relationships: is a type of extracellular matrix [GO:0031012] Definition: A collagen-containing extracellular matrix consisting of a thin layer of dense material found in various animal tissues interposed between the cells and the adjacent connective tissue. It consists of the basal lamina plus an associated layer of reticulin fibers. References: PMID:22505934, PMID:33605520, PMID:39223427